nuclear-transcribed mRNA catabolic process, RNase MRP-dependent [GO:0000294] (BP) References: PMID:14729943 Relationships: is a type of nuclear-transcribed mRNA catabolic process [GO:0000956] Also known as: nuclear mRNA catabolic process, endonucleolytic cleavage-dependent decay, nuclear-transcribed mRNA catabolic process, endonucleolytic cleavage-dependent decay Definition: A minor MRP-dependent nuclear-transcribed mRNA degradation pathway that begins with an endonucleolytic cleavage to generate unprotected ends.